{
  "term_id": "GO:0006357",
  "term_label": "regulation of transcription by RNA polymerase II",
  "gene": "UniProtKB:Q9H2W2",
  "gene_symbol": "MIXL1",
  "gene_name": "Homeobox protein MIXL1"
}